{
  "term_label": "hormone receptor binding",
  "term_id": "GO:0051427",
  "gene_name": "Natriuretic peptides B",
  "gene": "UniProtKB:P16860",
  "gene_symbol": "NPPB"
}